{
  "gene": "UniProtKB:Q9P2T1",
  "term_label": "Unknown molecular function",
  "gene_name": "GMP reductase 2",
  "term_id": "UNKNOWN:0001",
  "gene_symbol": "GMPR2"
}